{
  "gene": "UniProtKB:Q6ZRV2",
  "gene_symbol": "FAM83H",
  "term_label": "positive regulation of cell migration",
  "gene_name": "Protein FAM83H",
  "term_id": "GO:0030335"
}